R1/R6 cell differentiation [GO:0048052] (biological process) Relationships: is a type of compound eye photoreceptor cell differentiation [GO:0001751] Definition: The process in which relatively unspecialized cells acquire the specialized features of R1 and R6 photoreceptors. An example of this process is found in Drosophila melanogaster. Sources: GOC:jid